thiamine phosphate phosphatase activity [GO:0042131] (molecular function) Relationships: is a type of phosphatase activity [GO:0016791] Definition: Catalysis of the reaction: thiamine phosphate + H2O = thiamine + phosphate. Also known as: ThMPase, thiamin monophosphate phosphatase, thiamin phosphate phosphatase activity References: PMID:197075 Sources: RHEA:47948